cervix development [GO:0060067] (biological process) Sources: GOC:dph, GOC:ebc Also known as: Mullerian tract development Relationships: is a type of reproductive structure development [GO:0048608] Definition: The reproductive developmental process whose specific outcome is the progression of the cervix over time, from its formation to the mature structure.